{
  "term_id": "UNKNOWN:0001",
  "term_label": "Unknown molecular function",
  "gene": "UniProtKB:Q9BWT1",
  "gene_symbol": "CDCA7",
  "gene_name": "Cell division cycle-associated protein 7"
}